{
  "term_id": "GO:0007264",
  "gene_symbol": "ARHGEF28",
  "term_label": "small GTPase-mediated signal transduction",
  "gene": "UniProtKB:Q8N1W1",
  "gene_name": "Rho guanine nucleotide exchange factor 28"
}